{
  "gene_name": "Semaphorin-3G",
  "term_id": "GO:0030215",
  "gene": "UniProtKB:Q9NS98",
  "term_label": "semaphorin receptor binding",
  "gene_symbol": "SEMA3G"
}